{
  "term_label": "protein targeting to membrane",
  "term_id": "GO:0006612",
  "gene_name": "Palmitoyltransferase ZDHHC6",
  "gene_symbol": "ZDHHC6",
  "gene": "UniProtKB:Q9H6R6"
}